oxygen binding [GO:0019825] (MF) Definition: Binding to oxygen (O2). Sources: GOC:jl Also known as: cytochrome P450, cytochrome P450 activity Relationships: is a type of small molecule binding [GO:0036094]